{
  "term_label": "BMP receptor binding",
  "gene": "UniProtKB:Q6UXX9",
  "gene_name": "R-spondin-2",
  "gene_symbol": "RSPO2",
  "term_id": "GO:0070700"
}